6-phosphofructo-2-kinase activity [GO:0003873] (molecular function) Also known as: 6-phosphofructo-2-kinase (phosphorylating), 6-phosphofructose 2-kinase activity, ATP:D-fructose-6-phosphate 2-phosphotransferase activity, ATP:beta-D-fructose-6-phosphate 2-phosphotransferase activity, fructose 6-phosphate 2-kinase activity, phosphofructokinase 2 activity Sources: EC:2.7.1.105, RHEA:15653 Definition: Catalysis of the reaction: beta-D-fructose 6-phosphate + ATP = beta-D-fructose 2,6-bisphosphate + ADP + 2 H+. Relationships: is a type of phosphofructokinase activity [GO:0008443]